negative regulation of cell budding [GO:0045781] (biological process) Relationships: is a type of regulation of cell budding [GO:0007116]; is a type of negative regulation of cell division [GO:0051782]; is a type of negative regulation of asexual reproduction [GO:1903665]; negatively regulates cell budding [GO:0007114] Definition: Any process that stops, prevents, or reduces the frequency, rate or extent of cell budding. Sources: GOC:go_curators Also known as: negative regulation of budding, down regulation of cell budding, down-regulation of cell budding, downregulation of cell budding, inhibition of cell budding